{
  "gene": "UniProtKB:Q99470",
  "term_id": "UNKNOWN:0002",
  "gene_name": "Stromal cell-derived factor 2",
  "gene_symbol": "SDF2",
  "term_label": "Unknown biological process"
}